{
  "gene_symbol": "SNRPD3",
  "gene": "UniProtKB:P62318",
  "term_label": "U4 snRNP",
  "gene_name": "Small nuclear ribonucleoprotein Sm D3",
  "term_id": "GO:0005687"
}